{
  "gene_name": "Outer dense fiber protein 2",
  "gene": "UniProtKB:Q5BJF6",
  "gene_symbol": "ODF2",
  "term_id": "UNKNOWN:0001",
  "term_label": "Unknown molecular function"
}